{
  "gene_symbol": "FOXC1",
  "gene_name": "Forkhead box protein C1",
  "gene": "UniProtKB:Q12948",
  "term_id": "UNKNOWN:0003",
  "term_label": "Unknown cellular component"
}